{
  "term_id": "GO:0005739",
  "gene_symbol": "UNG",
  "gene_name": "Uracil-DNA glycosylase",
  "gene": "UniProtKB:P13051",
  "term_label": "mitochondrion"
}